{
  "term_label": "response to nicotine",
  "term_id": "GO:0035094",
  "gene_name": "Neuronal acetylcholine receptor subunit beta-3",
  "gene_symbol": "CHRNB3",
  "gene": "UniProtKB:Q05901"
}